{
  "term_label": "external side of plasma membrane",
  "gene_name": "Lymphocyte antigen 6 complex locus protein G6d",
  "gene_symbol": "LY6G6D",
  "term_id": "GO:0009897",
  "gene": "UniProtKB:O95868"
}